{
  "gene_name": "Beta-defensin 131B",
  "term_label": "Unknown molecular function",
  "gene": "UniProtKB:A0A096LNP1",
  "gene_symbol": "DEFB131B",
  "term_id": "UNKNOWN:0001"
}